alphaV-beta3 integrin-tumstatin complex [GO:0071114] (cellular component) References: PMID:12682293 Definition: A protein complex that consists of an alphaV-beta3 integrin complex bound to tumstatin, the NC1 domain of the alpha3 chain of type IV collagen. Relationships: is a type of GO:0098797 Also known as: ITGAV-ITGB3-COL4A3 complex